{
  "gene": "UniProtKB:Q14D33",
  "term_label": "detection of chemical stimulus involved in sensory perception of bitter taste",
  "gene_symbol": "RTP5",
  "term_id": "GO:0001580",
  "gene_name": "Receptor-transporting protein 5"
}